{
  "gene_name": "Caveolin-2",
  "term_label": "sarcolemma",
  "gene_symbol": "CAV2",
  "gene": "UniProtKB:P51636",
  "term_id": "GO:0042383"
}